{
  "gene": "UniProtKB:P01903",
  "term_label": "peptide antigen binding",
  "gene_symbol": "HLA-DRA",
  "gene_name": "HLA class II histocompatibility antigen, DR alpha chain",
  "term_id": "GO:0042605"
}